nephrocyte diaphragm assembly [GO:0036059] (BP) Relationships: is a type of GO:0034333; is a type of GO:0036058 References: PMID:18971929 Sources: GOC:mtg_kidney_jan10, GOC:sart Definition: The aggregation, arrangement and bonding together of a set of components to form a nephrocyte diaphragm, a specialized cell-cell junction found between nephrocytes of the insect kidney.